{
  "term_id": "UNKNOWN:0003",
  "gene_name": "Humanin-like 9",
  "gene": "UniProtKB:P0CJ76",
  "gene_symbol": "MTRNR2L9",
  "term_label": "Unknown cellular component"
}